{
  "gene_symbol": "WNT16",
  "term_label": "extracellular space",
  "term_id": "GO:0005615",
  "gene": "UniProtKB:Q9UBV4",
  "gene_name": "Protein Wnt-16"
}